phosphatidylethanolamine N-methyltransferase activity [GO:0004608] (molecular function) Definition: Catalysis of the reaction: S-adenosyl-L-methionine + phosphatidylethanolamine = S-adenosyl-L-homocysteine + H+ + phosphatidyl-N-methylethanolamine. Sources: EC:2.1.1.17, RHEA:11164 Also known as: LMTase activity, PEMT, S-adenosyl-L-methionine:phosphatidylethanolamine N-methyltransferase activity, lipid methyl transferase activity, phosphatidylethanolamine methyltransferase activity, phosphatidylethanolamine-N-methylase activity, phosphatidylethanolamine-S-adenosylmethionine methyltransferase activity Relationships: is_a N-methyltransferase activity [GO:0008170]; is a type of S-adenosylmethionine-dependent methyltransferase activity [GO:0008757]